{
  "term_label": "nucleus",
  "term_id": "GO:0005634",
  "gene_name": "Aurora kinase B",
  "gene": "UniProtKB:Q96GD4",
  "gene_symbol": "AURKB"
}